monosaccharide binding [GO:0048029] (MF) Subtypes: galactose binding [GO:0005534], GO:0005536, GO:0005537, GO:0031418, GO:0033222, rhamnose binding [GO:0033296], GO:0042806, fructose binding [GO:0070061], L-arabinofuranose binding [GO:2001084] Relationships: is a type of carbohydrate binding [GO:0030246]; is a type of small molecule binding [GO:0036094] Sources: GOC:jid Definition: Binding to a monosaccharide. Monosaccharides are the simplest carbohydrates; they are polyhydroxy aldehydes H[CH(OH)]nC(=O)H or polyhydroxy ketones H[CHOH]nC(=O)[CHOH]mH with three or more carbon atoms. They form the constitutional repeating units of oligo- and polysaccharides.